{
  "gene_symbol": "L1CAM",
  "term_id": "GO:0005886",
  "gene": "UniProtKB:P32004",
  "term_label": "plasma membrane",
  "gene_name": "Neural cell adhesion molecule L1"
}